regulation of neutrophil degranulation [GO:0043313] (biological process) Definition: Any process that modulates the frequency, rate, or extent of neutrophil degranulation. Also known as: regulation of neutrophil granule exocytosis Subtypes: negative regulation of neutrophil degranulation [GO:0043314], positive regulation of neutrophil degranulation [GO:0043315] Sources: ISBN:0781735149 Relationships: is a type of regulation of myeloid leukocyte mediated immunity [GO:0002886]; is a type of regulation of leukocyte degranulation [GO:0043300]; is a type of GO:0050776; regulates neutrophil degranulation [GO:0043312]